{
  "term_label": "protein kinase binding",
  "gene_name": "Inhibitor of Bruton tyrosine kinase",
  "gene": "UniProtKB:Q9P2D0",
  "gene_symbol": "IBTK",
  "term_id": "GO:0019901"
}